{
  "term_label": "cholesterol homeostasis",
  "gene": "UniProtKB:P06858",
  "gene_name": "Lipoprotein lipase",
  "gene_symbol": "LPL",
  "term_id": "GO:0042632"
}